{
  "term_label": "Unknown biological process",
  "term_id": "UNKNOWN:0002",
  "gene": "UniProtKB:Q8N4C9",
  "gene_symbol": "C17orf78",
  "gene_name": "Uncharacterized protein C17orf78"
}